enucleate erythrocyte differentiation [GO:0043353] (biological process) Also known as: enucleate RBC differentiation, enucleate red blood cell differentiation Sources: GOC:go_curators Definition: The process in which a myeloid precursor cell acquires specialized features of an erythrocyte without a nucleus. An example of this process is found in Mus musculus. Relationships: is_a erythrocyte differentiation [GO:0030218]